{
  "gene_symbol": "TOMM70",
  "term_id": "GO:0030943",
  "gene": "UniProtKB:O94826",
  "term_label": "mitochondrion targeting sequence binding",
  "gene_name": "Mitochondrial import receptor subunit TOM70"
}